{
  "term_label": "plasma membrane",
  "term_id": "GO:0005886",
  "gene_symbol": "OR51J1",
  "gene_name": "Olfactory receptor 51J1",
  "gene": "UniProtKB:Q9H342"
}